{
  "term_label": "Unknown molecular function",
  "term_id": "UNKNOWN:0001",
  "gene": "UniProtKB:P15954",
  "gene_symbol": "COX7C",
  "gene_name": "Cytochrome c oxidase subunit 7C, mitochondrial"
}